{
  "term_id": "GO:0044331",
  "gene_symbol": "FAT2",
  "gene_name": "Protocadherin Fat 2",
  "gene": "UniProtKB:Q9NYQ8",
  "term_label": "cell-cell adhesion mediated by cadherin"
}